{
  "term_id": "GO:0051225",
  "gene_name": "Gamma-tubulin complex component 5",
  "gene_symbol": "TUBGCP5",
  "gene": "UniProtKB:Q96RT8",
  "term_label": "spindle assembly"
}